S-adenosylhomocysteine metabolic process [GO:0046498] (biological process) Definition: The chemical reactions and pathways involving S-adenosylhomocysteine; the L-enantiomer is formed from S-adenosylmethionine and is a strong inhibitor of S-adenosylmethionine-mediated methylation reactions. It can be cleaved to form adenosine and homocysteine. Sources: ISBN:0198506732 Also known as: S-adenosylhomocysteine metabolism Relationships: is a type of modified amino acid metabolic process [GO:0006575]; is a type of sulfur compound metabolic process [GO:0006790]; is a type of purine ribonucleoside metabolic process [GO:0046128]; is a type of L-amino acid metabolic process [GO:0170033]; is a type of non-proteinogenic amino acid metabolic process [GO:0170041] Subtypes: GO:0019510